{
  "gene_symbol": "IL1RN",
  "gene_name": "Interleukin-1 receptor antagonist protein",
  "term_label": "negative regulation of interleukin-1-mediated signaling pathway",
  "gene": "UniProtKB:P18510",
  "term_id": "GO:2000660"
}